calyx of Held [GO:0044305] (cellular component) Definition: The terminal specialization of a calyciferous axon which forms large synapses in the mammalian auditory central nervous system. References: PMID:11823805 Sources: NIF_Subcellular:sao1684283879 Relationships: is a type of axon terminus [GO:0043679]